arbutin transmembrane transporter activity [GO:0042951] (molecular function) Definition: Enables the transfer of arbutin, a glycoside found in the bearberry and related plants which has been used to treat urinary-tract diseases, from one side of a membrane to the other. References: PMID:19965875 Sources: GOC:jl, GOC:mtg_transport Relationships: is a type of GO:0015573; is part of arbutin transport [GO:0042949]